{
  "term_id": "GO:0042645",
  "gene_name": "Transcription factor A, mitochondrial",
  "term_label": "mitochondrial nucleoid",
  "gene": "UniProtKB:Q00059",
  "gene_symbol": "TFAM"
}